{
  "term_id": "GO:0003735",
  "gene_symbol": "RPS29",
  "term_label": "structural constituent of ribosome",
  "gene_name": "Small ribosomal subunit protein uS14",
  "gene": "UniProtKB:P62273"
}